sophorose transport [GO:2001087] (biological process) Definition: The directed movement of a sophoroseacetate into, out of or within a cell, or between cells, by means of some agent such as a transporter or pore. Sources: GOC:mengo_curators Relationships: is a type of disaccharide transport [GO:0015766]